{
  "gene_symbol": "PPA1",
  "gene": "UniProtKB:Q15181",
  "term_label": "mitochondrion",
  "gene_name": "Inorganic pyrophosphatase",
  "term_id": "GO:0005739"
}